{
  "gene_symbol": "SMG6",
  "term_label": "telomerase holoenzyme complex",
  "gene": "UniProtKB:Q86US8",
  "term_id": "GO:0005697",
  "gene_name": "Telomerase-binding protein EST1A"
}